histone H2A deubiquitinase activity [GO:0140950] (MF) References: PMID:18226187, PMID:20436459 Definition: A histone deubiquitinase that cleaves ubiquitin from a histone H2A protein to which it is conjugated. Relationships: is a type of GO:0140934 Also known as: histone H2A deubiquitination